{
  "gene": "UniProtKB:Q7Z5P4",
  "term_label": "Unknown biological process",
  "gene_name": "17-beta-hydroxysteroid dehydrogenase 13",
  "term_id": "UNKNOWN:0002",
  "gene_symbol": "HSD17B13"
}